{
  "term_label": "natural killer cell mediated immunity",
  "term_id": "GO:0002228",
  "gene_symbol": "KLRD1",
  "gene": "UniProtKB:Q13241",
  "gene_name": "Natural killer cells antigen CD94"
}